{
  "gene": "UniProtKB:Q9UBL9",
  "gene_symbol": "P2RX2",
  "term_label": "extracellularly ATP-gated monoatomic cation channel activity",
  "term_id": "GO:0004931",
  "gene_name": "P2X purinoceptor 2"
}